{
  "gene_name": "Intraflagellar transport protein 172 homolog",
  "term_label": "Unknown molecular function",
  "gene_symbol": "IFT172",
  "term_id": "UNKNOWN:0001",
  "gene": "UniProtKB:Q9UG01"
}